{
  "term_label": "P-body",
  "gene_name": "m7GpppX diphosphatase",
  "gene": "UniProtKB:Q96C86",
  "gene_symbol": "DCPS",
  "term_id": "GO:0000932"
}